{
  "term_label": "organelle fusion",
  "gene_symbol": "VPS11",
  "gene_name": "Vacuolar protein sorting-associated protein 11 homolog",
  "term_id": "GO:0048284",
  "gene": "UniProtKB:Q9H270"
}